{
  "gene_symbol": "ZBBX",
  "term_label": "Unknown biological process",
  "gene_name": "Zinc finger B-box domain-containing protein 1",
  "gene": "UniProtKB:A8MT70",
  "term_id": "UNKNOWN:0002"
}